{
  "gene_symbol": "PRKCI",
  "term_id": "GO:0004674",
  "gene": "UniProtKB:P41743",
  "term_label": "protein serine/threonine kinase activity",
  "gene_name": "Protein kinase C iota type"
}